{
  "gene": "UniProtKB:Q9P2H0",
  "gene_name": "Centrosomal protein of 126 kDa",
  "term_id": "UNKNOWN:0001",
  "gene_symbol": "CEP126",
  "term_label": "Unknown molecular function"
}